{
  "gene_name": "Sorting and assembly machinery component 50 homolog",
  "gene_symbol": "SAMM50",
  "term_label": "SAM complex",
  "gene": "UniProtKB:Q9Y512",
  "term_id": "GO:0001401"
}